{
  "gene_name": "Shieldin complex subunit 3",
  "gene_symbol": "SHLD3",
  "term_id": "GO:2000042",
  "gene": "UniProtKB:Q6ZNX1",
  "term_label": "negative regulation of double-strand break repair via homologous recombination"
}